renal capsule formation [GO:0072129] (biological process) Relationships: is a type of anatomical structure formation involved in morphogenesis [GO:0048646]; is part of renal capsule morphogenesis [GO:0072128] Subtypes: mesonephric capsule formation [GO:0061287], metanephric capsule formation [GO:0072266] Sources: GOC:mtg_kidney_jan10 Definition: The developmental process pertaining to the initial formation of a renal capsule from unspecified parts. The renal capsule is the tough fibrous layer surrounding the kidney, covered in a thick layer of perinephric adipose tissue. It provides some protection from trauma and damage. During development, it comprises a single layer of flattened cells that lie just above the cortical stroma and the condensed mesenchyme of the nephrogenic zone. It is in this region that the early stages of nephron induction and formation of new generations ureteric bud branches occur, as the kidney expands.